{
  "gene_name": "Claudin-14",
  "gene": "UniProtKB:O95500",
  "gene_symbol": "CLDN14",
  "term_id": "GO:0005923",
  "term_label": "bicellular tight junction"
}